{
  "gene_symbol": "TUBB1",
  "term_label": "structural constituent of cytoskeleton",
  "term_id": "GO:0005200",
  "gene_name": "Tubulin beta-1 chain",
  "gene": "UniProtKB:Q9H4B7"
}